{
  "gene_symbol": "KRT33B",
  "term_label": "keratin filament",
  "gene": "UniProtKB:Q14525",
  "term_id": "GO:0045095",
  "gene_name": "Keratin, type I cuticular Ha3-II"
}